{
  "term_label": "cytoplasm",
  "gene_symbol": "PCBP1",
  "gene": "UniProtKB:Q15365",
  "term_id": "GO:0005737",
  "gene_name": "Poly(rC)-binding protein 1"
}